zoospore encystment on host [GO:0075218] (biological process) Sources: GOC:pamgo_curators Definition: The physiological, developmental and morphological changes that occur in a symbiont zoospore during the process of its encystment. Encystment means to enter a state of essentially suspended animation in which the spore is protected by an outer coating and remains immobile and inactive until favorable conditions for growth occur again. The host is defined as the larger of the organisms involved in a symbiotic interaction. Regulation: regulated by modulation of zoospore encystment on host [GO:0075219]; positively regulated by positive regulation of zoospore encystment on host [GO:0075220]; negatively regulated by negative regulation of zoospore encystment on host [GO:0075221] Relationships: is a type of GO:0075214